regulation of male mating behavior [GO:1902435] (biological process) Definition: Any process that modulates the frequency, rate or extent of male mating behavior. References: PMID:24089208 Sources: GOC:TermGenie Relationships: is a type of regulation of behavior [GO:0050795]; is a type of GO:2000241; regulates male mating behavior [GO:0060179] Subtypes: regulation of turning behavior involved in mating [GO:0061094], GO:1902436, positive regulation of male mating behavior [GO:1902437]